symbiont-mediated suppression of host complement activation by recruitment of complement control protein [GO:0141117] (biological process) Definition: A process by which a symbiont prevents the activation of host complement by binding a soluble complement control protein (CCP) of the host and recruiting it to the microbe surface. The normal role of CCPs is to prevent complement activation on 'self' cellular targets. When soluble CCPs are recuited to the surface of a microbe, the complement fails to activate. References: PMID:17513779, PMID:22540535, PMID:24129254, PMID:27304426 Also known as: suppression of complement activation by another organism by recruitment of complement control protein, suppression of complement activation by another organism by recuitement of complement control protein Relationships: is a type of symbiont-mediated suppression of host complement activation [GO:0042784]